{
  "gene": "UniProtKB:Q49SQ1",
  "gene_symbol": "GPR33",
  "term_id": "GO:0007200",
  "term_label": "phospholipase C-activating G protein-coupled receptor signaling pathway",
  "gene_name": "Probable G-protein coupled receptor 33"
}